{
  "gene": "UniProtKB:Q8TEU7",
  "gene_name": "Rap guanine nucleotide exchange factor 6",
  "gene_symbol": "RAPGEF6",
  "term_label": "neuron projection development",
  "term_id": "GO:0031175"
}